{
  "gene": "UniProtKB:Q12778",
  "term_id": "GO:0000981",
  "gene_symbol": "FOXO1",
  "gene_name": "Forkhead box protein O1",
  "term_label": "DNA-binding transcription factor activity, RNA polymerase II-specific"
}